{
  "term_label": "Unknown cellular component",
  "gene_name": "Olfactory receptor 11H7",
  "gene_symbol": "OR11H7",
  "gene": "UniProtKB:Q8NGC8",
  "term_id": "UNKNOWN:0003"
}